{
  "gene_name": "RNA-binding protein MEX3D",
  "gene": "UniProtKB:Q86XN8",
  "gene_symbol": "MEX3D",
  "term_id": "UNKNOWN:0001",
  "term_label": "Unknown molecular function"
}